{
  "gene": "UniProtKB:P10589",
  "gene_name": "COUP transcription factor 1",
  "term_id": "GO:0000122",
  "term_label": "negative regulation of transcription by RNA polymerase II",
  "gene_symbol": "NR2F1"
}